{
  "gene": "UniProtKB:Q8TC17",
  "term_id": "GO:0005737",
  "gene_symbol": "GRAPL",
  "term_label": "cytoplasm",
  "gene_name": "GRB2-related adapter protein-like"
}